{
  "term_id": "UNKNOWN:0001",
  "term_label": "Unknown molecular function",
  "gene_symbol": "C21orf58",
  "gene": "UniProtKB:P58505",
  "gene_name": "Uncharacterized protein C21orf58"
}